{
  "term_id": "GO:0005737",
  "gene": "UniProtKB:Q86V97",
  "gene_name": "Kelch repeat and BTB domain-containing protein 6",
  "term_label": "cytoplasm",
  "gene_symbol": "KBTBD6"
}